leaf phyllotactic patterning [GO:0060772] (biological process) Definition: The radial pattern formation process that results in the formation of leaf primordia around the center of a shoot apical meristem. Sources: GOC:dph, GOC:sdb_2009, GOC:tb Relationships: is a type of phyllotactic patterning [GO:0060771]